{
  "term_label": "Golgi apparatus",
  "gene_name": "Ras-related protein Rab-27B",
  "term_id": "GO:0005794",
  "gene_symbol": "RAB27B",
  "gene": "UniProtKB:O00194"
}